{
  "term_label": "Unknown biological process",
  "gene": "UniProtKB:Q9NRG1",
  "gene_name": "Phosphoribosyltransferase domain-containing protein 1",
  "term_id": "UNKNOWN:0002",
  "gene_symbol": "PRTFDC1"
}